{
  "gene": "UniProtKB:Q9NZI5",
  "term_id": "GO:0000978",
  "gene_name": "Grainyhead-like protein 1 homolog",
  "gene_symbol": "GRHL1",
  "term_label": "RNA polymerase II cis-regulatory region sequence-specific DNA binding"
}